glutathione-disulfide reductase (NADPH) activity [GO:0004362] (molecular function) References: PMID:36771108 Sources: RHEA:11740 Relationships: is a type of glutathione disulfide oxidoreductase activity [GO:0015038]; is a type of antioxidant activity [GO:0016209]; is a type of oxidoreductase activity, acting on a sulfur group of donors, NAD(P) as acceptor [GO:0016668] Also known as: glutathione reductase activity, glutathione-disulfide reductase (NADP) activity, glutathione-disulfide reductase activity, glutathione-disulphide reductase activity, GSH reductase activity, GSSG reductase activity, NADPH-GSSG reductase activity, NADPH-glutathione reductase activity, NADPH:oxidized-glutathione oxidoreductase activity, glutathione S-reductase activity, glutathione:NADP+ oxidoreductase activity, oxidized glutathione reduction Definition: Catalysis of the reaction: 2 glutathione + NADP+ = glutathione disulfide + NADPH + H+.